{
  "gene_symbol": "ANGPTL7",
  "term_label": "extracellular matrix",
  "gene": "UniProtKB:O43827",
  "term_id": "GO:0031012",
  "gene_name": "Angiopoietin-related protein 7"
}